{
  "gene": "UniProtKB:P40306",
  "gene_name": "Proteasome subunit beta type-10",
  "term_id": "GO:0005829",
  "term_label": "cytosol",
  "gene_symbol": "PSMB10"
}